negative regulation of sinapate ester biosynthetic process [GO:1903086] (biological process) Definition: Any process that stops, prevents or reduces the frequency, rate or extent of sinapate ester biosynthesis. Also known as: down regulation of sinapate ester anabolism, down regulation of sinapate ester biosynthesis, down regulation of sinapate ester biosynthetic process, down regulation of sinapate ester formation, down regulation of sinapate ester synthesis, down-regulation of sinapate ester anabolism, down-regulation of sinapate ester biosynthesis, down-regulation of sinapate ester biosynthetic process, down-regulation of sinapate ester formation, down-regulation of sinapate ester synthesis, downregulation of sinapate ester anabolism, downregulation of sinapate ester biosynthesis, downregulation of sinapate ester biosynthetic process, downregulation of sinapate ester formation, downregulation of sinapate ester synthesis, negative regulation of sinapate ester anabolism, negative regulation of sinapate ester biosynthesis, negative regulation of sinapate ester formation, negative regulation of sinapate ester synthesis, inhibition of sinapate ester anabolism, inhibition of sinapate ester biosynthesis, inhibition of sinapate ester biosynthetic process, inhibition of sinapate ester formation, inhibition of sinapate ester synthesis Relationships: is a type of negative regulation of secondary metabolite biosynthetic process [GO:1900377]; is a type of regulation of sinapate ester biosynthetic process [GO:1903085]; negatively regulates sinapate ester biosynthetic process [GO:0033525] References: PMID:11080161 Sources: GOC:TermGenie, GO_REF:0000058